{
  "gene_symbol": "IGHV8-51-1",
  "term_label": "antigen binding",
  "gene_name": "Probable non-functional immunoglobulin heavy variable 8-51-1",
  "term_id": "GO:0003823",
  "gene": "UniProtKB:P0DTE2"
}